{
  "gene_symbol": "SUN5",
  "gene_name": "SUN domain-containing protein 5",
  "gene": "UniProtKB:Q8TC36",
  "term_label": "Unknown biological process",
  "term_id": "UNKNOWN:0002"
}